{
  "gene_symbol": "MVB12A",
  "term_label": "cytosol",
  "gene_name": "Multivesicular body subunit 12A",
  "term_id": "GO:0005829",
  "gene": "UniProtKB:Q96EY5"
}